{
  "gene_name": "Uncharacterized protein LINC03042",
  "term_label": "Unknown molecular function",
  "term_id": "UNKNOWN:0001",
  "gene": "UniProtKB:Q6ZUL3",
  "gene_symbol": "LINC03042"
}